{
  "term_id": "GO:0090110",
  "gene": "UniProtKB:P53992",
  "gene_symbol": "SEC24C",
  "term_label": "COPII-coated vesicle cargo loading",
  "gene_name": "Protein transport protein Sec24C"
}